cis-trans isomerase activity [GO:0016859] (molecular function) Subtypes: GO:0003755, GO:0016034, carotenoid isomerase activity [GO:0046608], 2-chloro-4-carboxymethylenebut-2-en-1,4-olide isomerase activity [GO:0047466], GO:0047885, GO:0047907, linoleate isomerase activity [GO:0050058], maleate isomerase activity [GO:0050076], maleylpyruvate isomerase activity [GO:0050077], retinol isomerase activity [GO:0050251], 9,15,9'-tri-cis-zeta-carotene isomerase activity [GO:0090471], beta-carotene isomerase activity [GO:0106365] Definition: Catalysis of a reaction that interconverts cis and trans isomers. Atoms or groups are termed cis or trans to one another when they lie respectively on the same or on opposite sides of a reference plane identifiable as common among stereoisomers. Relationships: is a type of isomerase activity [GO:0016853] Sources: GOC:mah, ISBN:0198506732